{
  "gene_name": "Disintegrin and metalloproteinase domain-containing protein 32",
  "gene": "UniProtKB:Q8TC27",
  "term_label": "plasma membrane",
  "gene_symbol": "ADAM32",
  "term_id": "GO:0005886"
}